{
  "gene_symbol": "BAHD1",
  "term_id": "GO:0005677",
  "gene_name": "Bromo adjacent homology domain-containing 1 protein",
  "term_label": "chromatin silencing complex",
  "gene": "UniProtKB:Q8TBE0"
}